hippo signaling [GO:0035329] (biological process) Regulation: regulated by GO:0035330; negatively regulated by GO:0035331; positively regulated by positive regulation of hippo signaling [GO:0035332] Also known as: hippo signal transduction, hippo signaling pathway, SWH pathway, Salvador-Warts-Hippo signaling pathway, hippo signaling cascade, hippo signalling cascade References: PMID:17318211, PMID:18328423, PMID:36347846 Definition: An intracellular signaling cascade that starts with the activation of hippo (STK4/MST1 and STK3/MST2 in mammals and hpo kinase in Drosophila). Hippo then phosphorylates LATS1/2, which in turn phosphoylates the transcriptional co-activator YAP1 (yki in Drosophila), leading to its cytosolic retention and/or degradation. Relationships: is a type of intracellular signal transduction [GO:0035556]